{
  "term_id": "GO:1904263",
  "gene_name": "OTU domain-containing protein 5",
  "gene": "UniProtKB:Q96G74",
  "gene_symbol": "OTUD5",
  "term_label": "positive regulation of TORC1 signaling"
}